tendon formation [GO:0035992] (biological process) Relationships: is a type of GO:0048646; is part of tendon development [GO:0035989] Definition: The process that gives rise to a tendon. This process pertains to the initial formation of a tendon from unspecified parts. References: PMID:17567668 Sources: GOC:yaf, UBERON:0000043